{
  "gene_symbol": "BCS1L",
  "gene_name": "Mitochondrial chaperone BCS1",
  "gene": "UniProtKB:Q9Y276",
  "term_id": "UNKNOWN:0001",
  "term_label": "Unknown molecular function"
}